acid-thiol ligase activity [GO:0016878] (molecular function) Relationships: is a type of ligase activity, forming carbon-sulfur bonds [GO:0016877] Sources: EC:6.2.1.-, GOC:mah Definition: Catalysis of the joining of an acid and a thiol via a carbon-sulfur bond, with the concomitant hydrolysis of the diphosphate bond in ATP or a similar triphosphate. Subtypes: acetate-CoA ligase activity [GO:0003987], succinate-CoA ligase activity [GO:0004774], 2,3-dihydroxybenzoate--[aryl-carrier protein] ligase [GO:0008668], o-succinylbenzoate-CoA ligase activity [GO:0008756], GO:0008771, fatty acid ligase activity [GO:0015645], 4-coumarate-CoA ligase activity [GO:0016207], 2-oxo-delta3-4,5,5-trimethylcyclopentenylacetyl-CoA synthetase activity [GO:0018855], benzoyl acetate-CoA ligase activity [GO:0018856], GO:0018858, 4-hydroxybenzoate-CoA ligase activity [GO:0018859], anthranilate-CoA ligase activity [GO:0018860], 4-chlorobenzoate-CoA ligase activity [GO:0018861], acetoacetate-CoA ligase activity [GO:0030729], citronellyl-CoA ligase activity [GO:0034823], 6-carboxyhexanoate-CoA ligase activity [GO:0042410], acetate-CoA ligase (ADP-forming) activity [GO:0043758], 3-hydroxypropionyl-CoA synthetase activity [GO:0043955], D-alanine [D-alanyl carrier protein] ligase activity [GO:0047473], phenylacetate-CoA ligase activity [GO:0047475], 3-alpha,7-alpha-dihydroxy-5-beta-cholestanate-CoA ligase activity [GO:0047476], GO:0047541, GO:0047612, biotin-CoA ligase activity [GO:0047707], GO:0047747, GO:0047779, dicarboxylate-CoA ligase activity [GO:0047851], GO:0047948, malate-CoA ligase activity [GO:0050074], phytanate-CoA ligase activity [GO:0050197], GO:0050203, GO:0052686, (3R)-3-isopropenyl-6-oxoheptanoate:CoA ligase (ADP-forming) activity [GO:0052687], (3R)-3-isopropenyl-6-oxoheptanoate:CoA ligase (AMP-forming) activity [GO:0052688], pristanate-CoA ligase activity [GO:0070251]